cardiac septum morphogenesis [GO:0060411] (biological process) Relationships: is a type of anatomical structure morphogenesis [GO:0009653]; is part of cardiac chamber morphogenesis [GO:0003206]; is part of cardiac septum development [GO:0003279] Sources: GOC:dph, GOC:mtg_heart Definition: The process in which the anatomical structure of a cardiac septum is generated and organized. A cardiac septum is a partition that separates parts of the heart. Subtypes: outflow tract septum morphogenesis [GO:0003148], ventricular septum morphogenesis [GO:0060412], atrial septum morphogenesis [GO:0060413] Also known as: heart septum morphogenesis